antibacterial humoral response [GO:0019731] (biological process) Sources: GOC:go_curators, GOC:mtg_sensu Relationships: is a type of antimicrobial humoral response [GO:0019730]; is a type of GO:0042742 Subtypes: male-specific antibacterial humoral response [GO:0006962], induction of bacterial agglutination [GO:0043152] Definition: An immune response against bacteria mediated through a body fluid. Examples of this process are the antibacterial humoral responses in Mus musculus and Drosophila melanogaster.